{
  "gene_symbol": "TYRO3",
  "term_id": "GO:0043235",
  "term_label": "receptor complex",
  "gene": "UniProtKB:Q06418",
  "gene_name": "Tyrosine-protein kinase receptor TYRO3"
}